chemokine (C-C motif) ligand 4 production [GO:0071606] (biological process) Regulation: regulated by regulation of chemokine (C-C motif) ligand 4 production [GO:0071643]; negatively regulated by negative regulation of chemokine (C-C motif) ligand 4 production [GO:0071644]; positively regulated by GO:0071645 Relationships: is a type of chemokine production [GO:0032602] Also known as: macrophage inflammatory protein production, CCL4 production, MIP-1b production Definition: The appearance of chemokine (C-C motif) ligand 4 due to biosynthesis or secretion following a cellular stimulus, resulting in an increase in its intracellular or extracellular levels. Sources: GOC:add, GOC:rv